{
  "gene_symbol": "ROCK2",
  "gene_name": "Rho-associated protein kinase 2",
  "term_label": "cytoplasm",
  "gene": "UniProtKB:O75116",
  "term_id": "GO:0005737"
}